P4 peroxisome [GO:0019822] (cellular component) Note: Note that this peroxisome assembly pathway is described in the yeast Yarrowia lipolytica. See also the cellular component terms 'P1 peroxisome ; GO:0019819', 'P2 peroxisome ; GO:0019820', 'P3 peroxisome ; GO:0019821', 'P5 peroxisome ; GO:0019823', and 'P6 peroxisome ; GO:0019824'. Definition: A subform of peroxisome that corresponds to an intermediate in a peroxisome assembly pathway, which operates by conversion of peroxisomal subforms in the direction P1, P2 -> P3 -> P4 -> P5 -> P6. P4 peroxisomes are distinguished from the other subforms on the bases of buoyant density and protein content. Also known as: peroxisome vesicle Relationships: is a type of peroxisome [GO:0005777] References: PMID:10629216